{
  "gene": "UniProtKB:Q9H5J8",
  "term_label": "Unknown biological process",
  "term_id": "UNKNOWN:0002",
  "gene_name": "TATA box-binding protein-associated factor RNA polymerase I subunit D",
  "gene_symbol": "TAF1D"
}